{
  "term_label": "mitotic spindle disassembly",
  "gene": "UniProtKB:P55072",
  "gene_symbol": "VCP",
  "gene_name": "Transitional endoplasmic reticulum ATPase",
  "term_id": "GO:0051228"
}